{
  "gene_name": "Anaphase-promoting complex subunit 13",
  "gene": "UniProtKB:Q9BS18",
  "term_id": "GO:0070979",
  "gene_symbol": "ANAPC13",
  "term_label": "protein K11-linked ubiquitination"
}